redox taxis [GO:0009455] (biological process) Also known as: redoxtaxis, taxis in response to redox potential, taxis in response to redox stimulus Relationships: is a type of chemotaxis [GO:0006935]; is a type of GO:0009453; is a type of response to redox state [GO:0051775] References: PMID:11029423 Sources: GOC:jl Definition: The directed movement of a motile cell or organism in response to redox potential.